positive regulation of fatty acid beta-oxidation using acyl-CoA dehydrogenase [GO:1904737] (biological process) Relationships: is a type of positive regulation of fatty acid beta-oxidation [GO:0032000]; is a type of regulation of fatty acid beta-oxidation using acyl-CoA dehydrogenase [GO:1904735]; positively regulates GO:0033539 Definition: Any process that activates or increases the frequency, rate or extent of fatty acid beta-oxidation using acyl-CoA dehydrogenase. Also known as: up regulation of fatty acid beta-oxidation using acyl-CoA dehydrogenase, up-regulation of fatty acid beta-oxidation using acyl-CoA dehydrogenase, upregulation of fatty acid beta-oxidation using acyl-CoA dehydrogenase, activation of fatty acid beta-oxidation using acyl-CoA dehydrogenase References: PMID:25416781 Sources: GOC:TermGenie, GO_REF:0000058